nickel cation transport [GO:0015675] (biological process) Definition: The directed movement of nickel (Ni) cations into, out of or within a cell, or between cells, by means of some agent such as a transporter or pore. Sources: GOC:ai Relationships: is_a GO:0000041 Subtypes: nickel cation transmembrane transport [GO:0035444]